{
  "gene_name": "Scinderin",
  "term_label": "actin polymerization or depolymerization",
  "gene": "UniProtKB:Q9Y6U3",
  "gene_symbol": "SCIN",
  "term_id": "GO:0008154"
}